{
  "term_id": "GO:0070695",
  "gene_name": "FHF complex subunit HOOK-interacting protein 1B",
  "gene": "UniProtKB:Q8N612",
  "gene_symbol": "FHIP1B",
  "term_label": "FHF complex"
}